{
  "gene_symbol": "RPL10A",
  "gene_name": "Large ribosomal subunit protein uL1",
  "term_id": "GO:0003723",
  "gene": "UniProtKB:P62906",
  "term_label": "RNA binding"
}